{
  "gene": "UniProtKB:P35625",
  "term_id": "GO:0034097",
  "gene_name": "Metalloproteinase inhibitor 3",
  "gene_symbol": "TIMP3",
  "term_label": "response to cytokine"
}